{
  "gene_name": "DnaJ homolog subfamily B member 4",
  "gene": "UniProtKB:Q9UDY4",
  "term_id": "GO:0051087",
  "gene_symbol": "DNAJB4",
  "term_label": "protein-folding chaperone binding"
}